{
  "term_id": "GO:0051010",
  "gene": "UniProtKB:P43034",
  "gene_symbol": "PAFAH1B1",
  "gene_name": "Platelet-activating factor acetylhydrolase IB subunit beta",
  "term_label": "microtubule plus-end binding"
}